L-glyceraldehyde 3-phosphate reductase activity [GO:0103037] (molecular function) Relationships: is a type of GO:0016616 References: PMID:18620424 Sources: GOC:pz Definition: Catalysis of the reaction: sn-glycerol 3-phosphate + NADP = H+ + L-glyceraldehyde 3-phosphate + NADPH.